{
  "term_id": "GO:0090263",
  "gene_name": "Serine_threonine-protein kinase WNK2",
  "term_label": "positive regulation of canonical Wnt signaling pathway",
  "gene_symbol": "WNK2",
  "gene": "UniProtKB:Q9Y3S1"
}